{
  "gene_name": "Cytoskeleton-associated protein 2",
  "term_label": "negative regulation of microtubule depolymerization",
  "gene": "UniProtKB:Q8WWK9",
  "gene_symbol": "CKAP2",
  "term_id": "GO:0007026"
}